{
  "gene_symbol": "SDR16C5",
  "gene": "UniProtKB:Q8N3Y7",
  "term_label": "all-trans-retinol dehydrogenase (NAD+) activity",
  "gene_name": "Epidermal retinol dehydrogenase 2",
  "term_id": "GO:0004745"
}